{
  "term_label": "Unknown biological process",
  "gene_symbol": "SUSD2",
  "gene_name": "Sushi domain-containing protein 2",
  "gene": "UniProtKB:Q9UGT4",
  "term_id": "UNKNOWN:0002"
}